{
  "term_label": "regulation of glutamate receptor signaling pathway",
  "gene": "UniProtKB:Q9P0K9",
  "gene_name": "DOMON domain-containing protein FRRS1L",
  "gene_symbol": "FRRS1L",
  "term_id": "GO:1900449"
}